{
  "term_id": "GO:0007004",
  "gene": "UniProtKB:P27694",
  "gene_symbol": "RPA1",
  "term_label": "telomere maintenance via telomerase",
  "gene_name": "Replication protein A 70 kDa DNA-binding subunit"
}